{
  "term_label": "focal adhesion",
  "gene_name": "Caveolin-2",
  "gene_symbol": "CAV2",
  "gene": "UniProtKB:P51636",
  "term_id": "GO:0005925"
}